{
  "term_id": "GO:0043679",
  "gene_name": "Cadherin-8",
  "gene_symbol": "CDH8",
  "gene": "UniProtKB:P55286",
  "term_label": "axon terminus"
}